S-methylmethionine transport [GO:0015806] (biological process) Relationships: is a type of modified amino acid transport [GO:0072337]; is a type of sulfur compound transport [GO:0072348] Definition: The directed movement of S-methylmethionine into, out of or within a cell, or between cells, by means of some agent such as a transporter or pore. Sources: GOC:ai